{
  "term_id": "GO:0035459",
  "gene": "UniProtKB:A4D2H0",
  "gene_symbol": "CTAGE15",
  "term_label": "vesicle cargo loading",
  "gene_name": "cTAGE family member 15"
}